activin B complex [GO:0043510] (cellular component) Relationships: is a type of GO:0048180 Definition: A nonsteroidal regulator, composed of two covalently linked inhibin beta-B subunits (sometimes known as activin beta-B or activin/inhibin beta-B). Note: Note that the actions of the activin complex are the opposite of those of the inhibin complex, which is a dimer of an inhibin beta-A or inhibin beta-B subunit and a inhibin alpha subunit. See 'inhibin complex ; GO:0043511'. Sources: GOC:go_curators